{
  "gene_name": "Core histone macro-H2A.1",
  "term_label": "negative regulation of transcription by RNA polymerase II",
  "gene_symbol": "MACROH2A1",
  "gene": "UniProtKB:O75367",
  "term_id": "GO:0000122"
}